ubiquitin-dependent glycoprotein ERAD pathway [GO:0097466] (biological process) Relationships: is a type of glycoprotein catabolic process [GO:0006516]; is a type of ERAD pathway [GO:0036503]; is a type of GO:1904587 Definition: An ERAD pathway whereby endoplasmic reticulum (ER)-resident glycoproteins are targeted for degradation. Includes differential processing of the glycoprotein sugar chains, retrotranslocation to the cytosol and degradation by the ubiquitin-proteasome pathway. A glycoprotein is a compound in which a carbohydrate component is covalently bound to a protein component. Also known as: misfolded or incompletely synthesized glycoprotein catabolic process, ER-associated glycoprotein degradation, glycoprotein ERAD, gpERAD References: PMID:16079177 Sources: GOC:al, GOC:bf